{
  "term_label": "skeletal muscle contraction",
  "term_id": "GO:0003009",
  "gene": "UniProtKB:O15273",
  "gene_symbol": "TCAP",
  "gene_name": "Telethonin"
}